{
  "gene_name": "Lymphocyte transmembrane adapter 1",
  "term_id": "GO:0050851",
  "term_label": "antigen receptor-mediated signaling pathway",
  "gene_symbol": "LAX1",
  "gene": "UniProtKB:Q8IWV1"
}